{
  "term_id": "GO:0005886",
  "gene_symbol": "PCDHB3",
  "gene_name": "Protocadherin beta-3",
  "gene": "UniProtKB:Q9Y5E6",
  "term_label": "plasma membrane"
}